{
  "term_id": "UNKNOWN:0002",
  "gene": "UniProtKB:Q53HC0",
  "gene_name": "Coiled-coil domain-containing protein 92",
  "term_label": "Unknown biological process",
  "gene_symbol": "CCDC92"
}